{
  "gene": "UniProtKB:B5MCN3",
  "gene_symbol": "SEC14L6",
  "term_id": "UNKNOWN:0002",
  "gene_name": "Putative SEC14-like protein 6",
  "term_label": "Unknown biological process"
}